renal vesicle development [GO:0072087] (biological process) Sources: GOC:mtg_kidney_jan10 Definition: The process whose specific outcome is the progression of the renal vesicle over time, from its formation to the mature structure. An epithelium is a tissue that covers the internal or external surfaces of an anatomical structure. The renal vesicle is the primordial structure of the nephron epithelium, and is formed by the condensation of mesenchymal cells. Relationships: is a type of kidney epithelium development [GO:0072073]; is part of GO:0072009